{
  "gene_symbol": "GID8",
  "gene": "UniProtKB:Q9NWU2",
  "term_label": "protein-macromolecule adaptor activity",
  "gene_name": "Glucose-induced degradation protein 8 homolog",
  "term_id": "GO:0030674"
}